{
  "term_label": "nuclear receptor activity",
  "gene_name": "Nuclear receptor subfamily 1 group D member 2",
  "gene": "UniProtKB:Q14995",
  "term_id": "GO:0004879",
  "gene_symbol": "NR1D2"
}